apical cortex [GO:0045179] (cellular component) Sources: GOC:bf Definition: The region that lies just beneath the plasma membrane on the apical edge of a cell. Subtypes: apicomedial cortex [GO:0106037] Relationships: is a type of cell cortex region [GO:0099738]; is part of GO:0045177